adenyl nucleotide binding [GO:0030554] (molecular function) Sources: ISBN:0198506732 Relationships: is a type of purine nucleotide binding [GO:0017076] Subtypes: adenyl deoxyribonucleotide binding [GO:0032558], GO:0032559, NADP binding [GO:0050661], NAD binding [GO:0051287] Definition: Binding to an adenyl nucleotide, an adenosine esterified with (ortho)phosphate.